{
  "term_id": "GO:0032588",
  "gene": "UniProtKB:Q96N21",
  "term_label": "trans-Golgi network membrane",
  "gene_symbol": "TEPSIN",
  "gene_name": "AP-4 complex accessory subunit Tepsin"
}